{
  "gene_name": "General transcription factor 3C polypeptide 3",
  "term_label": "transcription factor TFIIIC complex",
  "gene_symbol": "GTF3C3",
  "term_id": "GO:0000127",
  "gene": "UniProtKB:Q9Y5Q9"
}